{
  "gene": "UniProtKB:Q6AI14",
  "term_label": "plasma membrane",
  "term_id": "GO:0005886",
  "gene_symbol": "SLC9A4",
  "gene_name": "Sodium_hydrogen exchanger 4"
}